{
  "gene_name": "Putative ubiquitin carboxyl-terminal hydrolase 41",
  "gene": "UniProtKB:Q3LFD5",
  "term_id": "UNKNOWN:0003",
  "gene_symbol": "USP41",
  "term_label": "Unknown cellular component"
}